{
  "gene": "UniProtKB:A6NEE1",
  "term_label": "Unknown cellular component",
  "term_id": "UNKNOWN:0003",
  "gene_name": "Pleckstrin homology domain-containing family D member 1",
  "gene_symbol": "PLEKHD1"
}